regulation of inflammasome-mediated signaling pathway [GO:0141085] (biological process) Definition: Any process that modulates the frequency, rate or extent of an inflammasome-mediated signaling pathway. References: PMID:33467177 Also known as: regulation of inflammasome-mediated signal transduction Relationships: is a type of regulation of cytoplasmic pattern recognition receptor signaling pathway [GO:0039531]; regulates inflammasome-mediated signaling pathway [GO:0141084] Subtypes: GO:0141086, positive regulation of inflammasome-mediated signaling pathway [GO:0141087]